{
  "term_label": "RNA polymerase II, core complex",
  "term_id": "GO:0005665",
  "gene_name": "DNA-directed RNA polymerases I, II, and III subunit RPABC3",
  "gene": "UniProtKB:P52434",
  "gene_symbol": "POLR2H"
}